mitotic sister chromatid cohesion, telomeric [GO:0099404] (biological process) Definition: The cell cycle process in which telomeres of sister chromatids are joined during mitosis. Relationships: is a type of mitotic sister chromatid cohesion [GO:0007064] Also known as: mitotic sister chromatid cohesion at telomere, sister chromatid cohesion at telomere at mitosis, telomeric mitotic sister chromatin cohesion References: PMID:26373281 Sources: GOC:BHF, GOC:BHF_telomere, GOC:mah, GOC:rph